{
  "gene_symbol": "ST3GAL6",
  "term_label": "sialyltransferase activity",
  "term_id": "GO:0008373",
  "gene": "UniProtKB:Q9Y274",
  "gene_name": "Type 2 lactosamine alpha-2,3-sialyltransferase"
}